{
  "term_id": "GO:0015629",
  "gene_symbol": "FSCN3",
  "gene": "UniProtKB:Q9NQT6",
  "gene_name": "Fascin-3",
  "term_label": "actin cytoskeleton"
}